{
  "gene_symbol": "GJB6",
  "gene_name": "Gap junction beta-6 protein",
  "gene": "UniProtKB:O95452",
  "term_label": "gap junction channel activity",
  "term_id": "GO:0005243"
}